lumenal side of plastid thylakoid membrane [GO:0098571] (CC) Sources: GOC:dos Definition: The side (leaflet) of the plastid thylakoid membrane that faces the lumen, and any proteins embedded in it or loosely bound to its surface. Relationships: is a type of side of membrane [GO:0098552]; is part of plastid thylakoid membrane [GO:0055035]